{
  "gene": "UniProtKB:Q6PL18",
  "term_id": "GO:0006334",
  "term_label": "nucleosome assembly",
  "gene_symbol": "ATAD2",
  "gene_name": "ATPase family AAA domain-containing protein 2"
}